{
  "gene_name": "Testis-specific serine_threonine-protein kinase 1",
  "gene": "UniProtKB:Q9BXA7",
  "term_id": "GO:0007286",
  "term_label": "spermatid development",
  "gene_symbol": "TSSK1B"
}